{
  "term_id": "GO:0005886",
  "gene_name": "Clathrin light chain A",
  "term_label": "plasma membrane",
  "gene_symbol": "CLTA",
  "gene": "UniProtKB:P09496"
}